{
  "term_id": "GO:0005886",
  "gene_name": "E3 ubiquitin-protein ligase CBL",
  "gene": "UniProtKB:P22681",
  "term_label": "plasma membrane",
  "gene_symbol": "CBL"
}